{
  "gene": "UniProtKB:O60336",
  "term_label": "Unknown molecular function",
  "gene_name": "Mitogen-activated protein kinase-binding protein 1",
  "term_id": "UNKNOWN:0001",
  "gene_symbol": "MAPKBP1"
}